{
  "term_label": "spliceosomal snRNP assembly",
  "gene_symbol": "GEMIN7",
  "term_id": "GO:0000387",
  "gene": "UniProtKB:Q9H840",
  "gene_name": "Gem-associated protein 7"
}